{
  "gene": "UniProtKB:Q96GI7",
  "gene_name": "Protein FAM89A",
  "gene_symbol": "FAM89A",
  "term_id": "UNKNOWN:0003",
  "term_label": "Unknown cellular component"
}